mesonephric nephron tubule epithelial cell differentiation [GO:0061265] (biological process) Definition: The process in which relatively unspecialized cells acquire specialized structural and/or functional features that characterize the cells of the mesonephric nephron tubule as it progresses from its formation to the mature state. Regulation: regulated by regulation of mesonephric nephron tubule epithelial cell differentiation [GO:2000093]; negatively regulated by GO:2000094 Sources: GOC:mtg_kidney_jan10 Relationships: is a type of cell differentiation involved in mesonephros development [GO:0061208]; is a type of nephron tubule epithelial cell differentiation [GO:0072160]; is part of mesonephric nephron tubule development [GO:0061242]